{
  "gene_name": "BPI fold-containing family C protein",
  "gene_symbol": "BPIFC",
  "term_id": "GO:0005615",
  "term_label": "extracellular space",
  "gene": "UniProtKB:Q8NFQ6"
}